{
  "term_id": "GO:0042127",
  "gene_name": "Transcription factor JunB",
  "gene_symbol": "JUNB",
  "gene": "UniProtKB:P17275",
  "term_label": "regulation of cell population proliferation"
}